{
  "term_label": "neuron projection",
  "term_id": "GO:0043005",
  "gene_name": "Teneurin-1",
  "gene_symbol": "TENM1",
  "gene": "UniProtKB:Q9UKZ4"
}